{
  "term_label": "plasma membrane",
  "term_id": "GO:0005886",
  "gene_name": "Activin receptor type-1B",
  "gene_symbol": "ACVR1B",
  "gene": "UniProtKB:P36896"
}